{
  "gene_symbol": "PTPN2",
  "gene": "UniProtKB:P17706",
  "gene_name": "Tyrosine-protein phosphatase non-receptor type 2",
  "term_id": "GO:0019901",
  "term_label": "protein kinase binding"
}